cardioblast migration to the midline involved in heart field formation [GO:0060975] (biological process) Subtypes: cardiac muscle progenitor cell migration to the midline involved in heart field formation [GO:0003261], endocardial progenitor cell migration to the midline involved in heart field formation [GO:0003262] Relationships: is a type of cardioblast migration [GO:0003260]; is a type of cell migration to the midline involved in heart development [GO:0003318]; is part of convergent extension involved in organogenesis [GO:0060029] Sources: GOC:mtg_heart Also known as: cardiac progenitor cell midline migration, cardioblast midline convergence Definition: The orderly movement of a cardioblast toward the midline to form the heart field. A cardioblast is a cardiac precursor cell. It is a cell that has been committed to a cardiac fate, but will undergo more cell division rather than terminally differentiating.